chemokine (C-X-C motif) ligand 12 signaling pathway [GO:0038146] (biological process) Also known as: CXCL12 signaling pathway, SDF1 signaling pathway, stromal cell-derived factor-1 signaling pathway, CXCL12-activated CXCR7 signaling pathway Sources: GOC:nhn, GOC:signaling, Wikipedia:Stromal_cell-derived_factor-1 Relationships: is a type of chemokine-mediated signaling pathway [GO:0070098] Subtypes: GO:0038160 Definition: The series of molecular signals initiated by the binding of the chemokine CXCL12 to its receptor on the surface of a target cell, and ending with the regulation of a downstream cellular process, e.g. transcription.